purine nucleoside transmembrane transport [GO:0015860] (BP) Relationships: is a type of purine-containing compound transmembrane transport [GO:0072530]; is a type of nucleoside transmembrane transport [GO:1901642] Definition: The process in which a purine nucleoside is transported across a membrane. A purine nucleoside is a purine base covalently bonded to a ribose or deoxyribose sugar. Note: Note that this term is not intended for use in annotating lateral movement within membranes. Also known as: purine nucleoside transport, purine nucleoside membrane transport Sources: GOC:ai, GOC:vw